{
  "gene": "UniProtKB:Q03403",
  "gene_symbol": "TFF2",
  "term_label": "chemokine-mediated signaling pathway",
  "term_id": "GO:0070098",
  "gene_name": "Trefoil factor 2"
}